{
  "term_id": "GO:0051603",
  "gene": "UniProtKB:P09668",
  "gene_symbol": "CTSH",
  "gene_name": "Pro-cathepsin H",
  "term_label": "proteolysis involved in protein catabolic process"
}